{
  "gene_name": "Gilles de la Tourette syndrome chromosomal region candidate gene 1 protein",
  "gene": "UniProtKB:Q86UQ5",
  "gene_symbol": "GTSCR1",
  "term_label": "Unknown biological process",
  "term_id": "UNKNOWN:0002"
}